interleukin-1 binding [GO:0019966] (MF) Definition: Binding to interleukin-1. Also known as: IL-1 binding Sources: GOC:jl, ISBN:0198506732 Subtypes: interleukin-1 receptor antagonist activity [GO:0005152] Relationships: is a type of growth factor binding [GO:0019838]; is a type of cytokine binding [GO:0019955]